leukemia inhibitory factor signaling pathway involved in forebrain neuron fate commitment [GO:0022025] (biological process) Relationships: is_a leukemia inhibitory factor signaling pathway [GO:0048861]; is part of commitment of multipotent stem cells to neuronal lineage in forebrain [GO:0021898] Sources: GOC:cls, GOC:dgh, GOC:dph, GOC:jid, GOC:signaling Definition: The series of molecular signals initiated by the binding of leukemia inhibitory factor to its receptor on the surface of the target cell, that contributes to the commitment of a neuroblast to a neuronal fate. The neuron will reside in the forebrain. Also known as: leukemia inhibitory factor signalling pathway involved in forebrain neuron fate commitment